SCF-Ufo1/Pof10 ubiquitin ligase complex [GO:0097670] (cellular component) Relationships: is a type of SCF ubiquitin ligase complex [GO:0019005] References: PMID:14747994, PMID:15147268 Sources: GOC:jd, GOC:vw Definition: An SCF ubiquitin ligase complex in which the F-box protein is Ufo1 in S. cerevisiae (Pof10 in S. pombe).